{
  "gene_name": "Beta-defensin 129",
  "gene_symbol": "DEFB129",
  "term_id": "UNKNOWN:0003",
  "gene": "UniProtKB:Q9H1M3",
  "term_label": "Unknown cellular component"
}